{
  "term_id": "GO:0005634",
  "gene_symbol": "RFC2",
  "gene_name": "Replication factor C subunit 2",
  "gene": "UniProtKB:P35250",
  "term_label": "nucleus"
}